{
  "gene_symbol": "FLNA",
  "term_label": "Unknown molecular function",
  "gene_name": "Filamin-A",
  "term_id": "UNKNOWN:0001",
  "gene": "UniProtKB:P21333"
}